{
  "gene_name": "Zinc finger protein ZIC 1",
  "gene": "UniProtKB:Q15915",
  "term_id": "GO:0006357",
  "term_label": "regulation of transcription by RNA polymerase II",
  "gene_symbol": "ZIC1"
}